Fc-gamma receptor signaling pathway [GO:0038094] (biological process) Also known as: Fc-gamma receptor signalling pathway Definition: The series of molecular signals initiated by the binding of the Fc portion of immunoglobulin G (IgG) to an Fc-gamma receptor on the surface of a target cell, and ending with the regulation of a downstream cellular process, e.g. transcription. The Fc portion of an immunoglobulin is its C-terminal constant region. Subtypes: Fc-gamma receptor signaling pathway involved in phagocytosis [GO:0038096] References: PMID:11244038 Sources: GOC:phg Relationships: is a type of Fc receptor signaling pathway [GO:0038093]